phospholipase A2 activator activity [GO:0016005] (molecular function) Definition: Binds to and increases the activity of the enzyme phospholipase A2. Sources: GOC:ai Relationships: is a type of GO:0016004; positively regulates GO:0004623